type 2 metabotropic glutamate receptor binding [GO:0031799] (molecular function) Sources: GOC:mah, GOC:nln Also known as: type 2 metabotropic glutamate receptor ligand Relationships: is a type of G protein-coupled glutamate receptor binding [GO:0035256] Definition: Binding to a type 2 metabotropic glutamate receptor.